{
  "gene": "UniProtKB:E9PB15",
  "gene_symbol": "PTGES3L",
  "gene_name": "Putative protein PTGES3L",
  "term_id": "GO:0051087",
  "term_label": "protein-folding chaperone binding"
}